{
  "gene": "UniProtKB:Q5H9B9",
  "gene_name": "Putative BMP-2-inducible kinase-like protein",
  "term_id": "UNKNOWN:0001",
  "gene_symbol": "BMP2KL",
  "term_label": "Unknown molecular function"
}